olfactory bulb development [GO:0021772] (biological process) Definition: The progression of the olfactory bulb over time from its initial formation until its mature state. The olfactory bulb coordinates neuronal signaling involved in the perception of smell. It receives input from the sensory neurons and outputs to the olfactory cortex. Sources: GOC:cls, GOC:dgh, GOC:dph, GOC:jid, GO_REF:0000021 Relationships: is a type of GO:0048856; is part of GO:0021988